cell growth involved in cardiac muscle cell development [GO:0061049] (biological process) Regulation: regulated by GO:0061050; positively regulated by GO:0061051; negatively regulated by negative regulation of cell growth involved in cardiac muscle cell development [GO:0061052] Relationships: is a type of developmental cell growth [GO:0048588]; is part of GO:0003301; is part of cardiac muscle cell development [GO:0055013] Also known as: cardiac muscle cell hypertrophy, cardiomyocyte growth, heart muscle cell growth Sources: GOC:dph Subtypes: embryonic cardiac muscle cell growth involved in heart morphogenesis [GO:0003246] Definition: The growth of a cardiac muscle cell, where growth contributes to the progression of the cell over time from its initial formation to its mature state.